{
  "term_id": "GO:0005829",
  "term_label": "cytosol",
  "gene_symbol": "TRIM6",
  "gene": "UniProtKB:Q9C030",
  "gene_name": "Tripartite motif-containing protein 6"
}